cyclin B1-CDK1 complex [GO:0097125] (cellular component) Definition: A protein complex consisting of cyclin B1 and cyclin-dependent kinase 1 (CDK1). Cyclins are characterized by periodicity in protein abundance throughout the cell cycle. Cyclin-dependent kinases represent a family of serine/threonine protein kinases that become active upon binding to a cyclin regulatory partner. References: PMID:15935619 Sources: GOC:so Relationships: is a type of cyclin-dependent protein kinase holoenzyme complex [GO:0000307]